{
  "term_label": "intracellular calcium ion homeostasis",
  "gene_symbol": "ATP13A2",
  "term_id": "GO:0006874",
  "gene_name": "Polyamine-transporting ATPase 13A2",
  "gene": "UniProtKB:Q9NQ11"
}